{
  "gene_name": "Interleukin-34",
  "term_id": "GO:0045657",
  "term_label": "positive regulation of monocyte differentiation",
  "gene_symbol": "IL34",
  "gene": "UniProtKB:Q6ZMJ4"
}